{
  "gene_name": "Ras-related protein Rap-1b",
  "term_id": "GO:0005886",
  "gene_symbol": "RAP1B",
  "term_label": "plasma membrane",
  "gene": "UniProtKB:P61224"
}